{
  "gene_name": "Keratin-associated protein 10-8",
  "gene_symbol": "KRTAP10-8",
  "gene": "UniProtKB:P60410",
  "term_label": "Unknown biological process",
  "term_id": "UNKNOWN:0002"
}